trialkylsulfonium hydrolase activity [GO:0016802] (molecular function) Also known as: thioether hydrolase activity, trialkylsulphonium hydrolase activity Relationships: is a type of GO:0016801 Sources: EC:3.3.1.-, GOC:ai Subtypes: adenosylselenohomocysteinase activity [GO:0098604] Definition: Catalysis of the hydrolysis of a thioether bond, -S-.